lignan biosynthetic process [GO:0009807] (biological process) Definition: The chemical reactions and pathways resulting in the formation of lignans, any member of a class of plant metabolites related to lignins. Lignans are usually found as phenylpropanoid dimers in which the phenylpropanoid units are linked tail to tail and thus having a 2,3 dibenzylbutane skeleton, but higher oligomers can also exist. References: PMID:10074466 Sources: GOC:jl Also known as: lignan anabolism, lignan biosynthesis, lignan formation, lignan synthesis Relationships: is_a phenylpropanoid biosynthetic process [GO:0009699]; is a type of lignan metabolic process [GO:0009806] Subtypes: (-)-pinoresinol biosynthetic process [GO:1901599], GO:1901708, (+)-pinoresinol biosynthetic process [GO:1902126], GO:1902129, (+)-lariciresinol biosynthetic process [GO:1902132], (+)-secoisolariciresinol biosynthetic process [GO:1902135], (-)-secoisolariciresinol biosynthetic process [GO:1902138]